{
  "gene": "UniProtKB:Q8N3L3",
  "gene_name": "Beta-taxilin",
  "term_id": "UNKNOWN:0002",
  "term_label": "Unknown biological process",
  "gene_symbol": "TXLNB"
}